{
  "gene_symbol": "CFAP157",
  "gene_name": "Cilia- and flagella-associated protein 157",
  "gene": "UniProtKB:Q5JU67",
  "term_id": "GO:0036064",
  "term_label": "ciliary basal body"
}